{
  "gene_symbol": "PPP1R3D",
  "gene_name": "Protein phosphatase 1 regulatory subunit 3D",
  "term_id": "GO:0000164",
  "gene": "UniProtKB:O95685",
  "term_label": "protein phosphatase type 1 complex"
}